{
  "term_id": "GO:0031262",
  "term_label": "Ndc80 complex",
  "gene_name": "Kinetochore protein Spc24",
  "gene": "UniProtKB:Q8NBT2",
  "gene_symbol": "SPC24"
}